myo-inosose-2 dehydratase activity [GO:0050114] (molecular function) Relationships: is a type of hydro-lyase activity [GO:0016836] Also known as: 2,4,6/3,5-pentahydroxycyclohexanone hydro-lyase (3,5/4-trihydroxycyclohexa-1,2-dione-forming), 2,4,6/3,5-pentahydroxycyclohexanone hydro-lyase activity, inosose 2,3-dehydratase activity, ketoinositol dehydratase activity Definition: Catalysis of the reaction: 2,4,6/3,5-pentahydroxycyclohexanone = 3D-3,5/4-trihydroxycyclohexane-1,2-dione + H2O. Sources: EC:4.2.1.44, RHEA:14065